{
  "term_label": "Unknown molecular function",
  "gene_symbol": "CRELD2",
  "gene_name": "Protein disulfide isomerase CRELD2",
  "term_id": "UNKNOWN:0001",
  "gene": "UniProtKB:Q6UXH1"
}